{
  "gene_symbol": "CLASP2",
  "gene_name": "CLIP-associating protein 2",
  "gene": "UniProtKB:O75122",
  "term_id": "GO:0008017",
  "term_label": "microtubule binding"
}